 [oboInOwl#source]